{
  "gene_name": "Fructose-bisphosphate aldolase B",
  "term_id": "GO:0061609",
  "gene": "UniProtKB:P05062",
  "gene_symbol": "ALDOB",
  "term_label": "fructose-1-phosphate aldolase activity"
}